{
  "term_id": "GO:0005730",
  "term_label": "nucleolus",
  "gene": "UniProtKB:O75691",
  "gene_symbol": "UTP20",
  "gene_name": "Small subunit processome component 20 homolog"
}